{
  "gene": "UniProtKB:Q9HBW1",
  "term_label": "plasma membrane",
  "gene_symbol": "LRRC4",
  "gene_name": "Leucine-rich repeat-containing protein 4",
  "term_id": "GO:0005886"
}